{
  "gene_name": "Olfactory receptor 10X1",
  "gene_symbol": "OR10X1",
  "gene": "UniProtKB:Q8NGY0",
  "term_id": "UNKNOWN:0003",
  "term_label": "Unknown cellular component"
}